multicellular organismal movement [GO:0050879] (BP) Subtypes: GO:0010031, musculoskeletal movement [GO:0050881], GO:0071965 Relationships: is a type of multicellular organismal process [GO:0032501] Sources: GOC:dph, GOC:mtg_muscle, GOC:tb Definition: Any physiological process involved in changing the position of a multicellular organism or an anatomical part of a multicellular organism.